{
  "gene_name": "Actin, aortic smooth muscle",
  "gene": "UniProtKB:P62736",
  "term_label": "actin cytoskeleton",
  "gene_symbol": "ACTA2",
  "term_id": "GO:0015629"
}